{
  "gene": "UniProtKB:Q6UWI2",
  "term_id": "GO:0005769",
  "gene_symbol": "PARM1",
  "term_label": "early endosome",
  "gene_name": "Prostate androgen-regulated mucin-like protein 1"
}